{
  "term_id": "GO:0008474",
  "gene_symbol": "ABHD17A",
  "gene": "UniProtKB:Q96GS6",
  "term_label": "palmitoyl-(protein) hydrolase activity",
  "gene_name": "Alpha_beta hydrolase domain-containing protein 17A"
}